{
  "gene_symbol": "ZFAND4",
  "gene": "UniProtKB:Q86XD8",
  "term_id": "UNKNOWN:0001",
  "term_label": "Unknown molecular function",
  "gene_name": "AN1-type zinc finger protein 4"
}